{
  "gene": "UniProtKB:Q01484",
  "term_id": "GO:0044325",
  "gene_name": "Ankyrin-2",
  "term_label": "transmembrane transporter binding",
  "gene_symbol": "ANK2"
}